{
  "gene": "UniProtKB:P0DV75",
  "term_label": "Unknown molecular function",
  "gene_name": "Protein FAM90A18",
  "gene_symbol": "FAM90A18",
  "term_id": "UNKNOWN:0001"
}